flavone 3'-O-methyltransferase activity [GO:0102822] (molecular function) Relationships: is a type of GO:0008171; is_a S-adenosylmethionine-dependent methyltransferase activity [GO:0008757] Also known as: luteolin O-methyltransferase activity, quercetin 3'-O-methyltransferase activity Definition: Catalysis of the reaction: a 3'-hydroxyflavone + S-adenosyl-L-methionine = a 3'-methoxyflavone + H+ + S-adenosyl-L-homocysteine. Sources: RHEA:55332